{
  "term_label": "mitotic cell cycle",
  "gene_symbol": "CENPW",
  "term_id": "GO:0000278",
  "gene": "UniProtKB:Q5EE01",
  "gene_name": "Centromere protein W"
}